{
  "gene_symbol": "ACOT6",
  "term_id": "GO:0006637",
  "gene": "UniProtKB:Q3I5F7",
  "term_label": "acyl-CoA metabolic process",
  "gene_name": "Acyl-coenzyme A thioesterase 6"
}